fusion of virus membrane with host outer membrane [GO:0098997] (biological process) Also known as: viral envelope fusion, viral penetration via membrane fusion, viral envelope fusion with host outer membrane, fusion of viral membrane with host outer membrane, viral-cell fusion molecule activity Definition: Fusion of a viral membrane with the host cell outer membrane during viral entry. Relationships: is a type of fusion of virus membrane with host plasma membrane [GO:0019064] Sources: GOC:dos, VZ:3941